response to symbiotic bacterium [GO:0009609] (biological process) Sources: GOC:hb, ISBN:0198506732 Relationships: is a type of response to symbiont [GO:0009608]; is a type of response to bacterium [GO:0009617] Also known as: response to symbiotic bacteria Subtypes: detection of symbiotic bacterium [GO:0009604] Definition: Any process that results in a change in state or activity of a cell or an organism (in terms of movement, secretion, enzyme production, gene expression, etc.) as a result of a stimulus from a symbiotic bacterium, a bacterium living in close physical association with another organism.